{
  "gene": "UniProtKB:Q96E14",
  "term_id": "UNKNOWN:0001",
  "term_label": "Unknown molecular function",
  "gene_name": "RecQ-mediated genome instability protein 2",
  "gene_symbol": "RMI2"
}